response to farnesol [GO:0097307] (biological process) Definition: Any process that results in a change in state or activity of a cell or an organism (in terms of movement, secretion, enzyme production, gene expression, etc.) as a result of a farnesol stimulus. Sources: GOC:pr Subtypes: cellular response to farnesol [GO:0097308] Relationships: is a type of GO:0033993; is_a response to alcohol [GO:0097305]